{
  "term_id": "GO:0046982",
  "gene": "UniProtKB:P35638",
  "gene_symbol": "DDIT3",
  "term_label": "protein heterodimerization activity",
  "gene_name": "DNA damage-inducible transcript 3 protein"
}